{
  "term_id": "GO:0005634",
  "term_label": "nucleus",
  "gene_symbol": "H2AC6",
  "gene": "UniProtKB:Q93077",
  "gene_name": "Histone H2A type 1-C"
}